{
  "gene": "UniProtKB:Q8NGX5",
  "term_label": "olfactory receptor activity",
  "term_id": "GO:0004984",
  "gene_symbol": "OR10K1",
  "gene_name": "Olfactory receptor 10K1"
}